{
  "term_label": "cytoplasm",
  "gene_name": "UBX domain-containing protein 1",
  "gene": "UniProtKB:Q04323",
  "term_id": "GO:0005737",
  "gene_symbol": "UBXN1"
}